somatic muscle attachment to chitin-based cuticle [GO:0160175] (biological process) Definition: The developmental process in which a somatic muscle attaches to the chitin-based cuticle. In insects, this may occur via a specialized epithelial cell adherence to the chitinous extracellular matrix and to muscle cells through their basement membrane. Relationships: is a type of somatic muscle development [GO:0007525] References: PMID:35675426